glucosylceramide metabolic process [GO:0006678] (biological process) Subtypes: glucosylceramide biosynthetic process [GO:0006679], glucosylceramide catabolic process [GO:0006680] Also known as: glucosylceramide metabolism Sources: ISBN:0198506732 Relationships: is a type of glycosylceramide metabolic process [GO:0006677] Definition: The chemical reactions and pathways involving glucosylceramides, any compound formed by the replacement of the glycosidic hydroxyl group of a cyclic form of glucose by a ceramide group. They are neutral glycolipids containing equimolar amounts of fatty acid, glucose, and sphingosine or a sphingosine derivative.